intracellular iron ion homeostasis [GO:0006879] (biological process) Sources: GOC:ai, GOC:mah Subtypes: iron import into cell [GO:0033212] Also known as: iron homeostasis, cellular iron ion homeostasis Definition: A homeostatic process involved in the maintenance of a steady state level of iron ions within a cell. Relationships: is a type of intracellular monoatomic cation homeostasis [GO:0030003]; is a type of inorganic ion homeostasis [GO:0098771]